{
  "gene": "UniProtKB:Q16644",
  "gene_name": "MAP kinase-activated protein kinase 3",
  "gene_symbol": "MAPKAPK3",
  "term_label": "toll-like receptor signaling pathway",
  "term_id": "GO:0002224"
}